GDP-L-fucose metabolic process [GO:0046368] (biological process) Definition: The chemical reactions and pathways involving GDP-L-fucose, a substance composed of L-fucose in glycosidic linkage with guanosine diphosphate. Sources: GOC:ai Subtypes: GO:0042350 Also known as: GDP-L-fucose metabolism Relationships: is a type of nucleotide-sugar metabolic process [GO:0009225]